{
  "gene_name": "Receptor-type tyrosine-protein phosphatase H",
  "gene_symbol": "PTPRH",
  "gene": "UniProtKB:Q9HD43",
  "term_id": "GO:0004725",
  "term_label": "protein tyrosine phosphatase activity"
}